{
  "gene_symbol": "RNF181",
  "gene": "UniProtKB:Q9P0P0",
  "term_id": "GO:0005737",
  "gene_name": "E3 ubiquitin-protein ligase RNF181",
  "term_label": "cytoplasm"
}